{
  "term_id": "GO:0005840",
  "gene_symbol": "RPL13A",
  "term_label": "ribosome",
  "gene_name": "Large ribosomal subunit protein uL13",
  "gene": "UniProtKB:P40429"
}